{
  "term_label": "carbohydrate binding",
  "gene": "UniProtKB:O00182",
  "gene_name": "Galectin-9",
  "gene_symbol": "LGALS9",
  "term_id": "GO:0030246"
}